pectin binding [GO:0044589] (molecular function) Relationships: is a type of galacturonan binding [GO:0048028] Definition: Binding to pectin. Sources: GOC:mengo_curators, GOC:tt